{
  "gene": "UniProtKB:Q8TD57",
  "term_id": "GO:0097729",
  "term_label": "9+2 motile cilium",
  "gene_symbol": "DNAH3",
  "gene_name": "Dynein axonemal heavy chain 3"
}